protein localization to spindle pole body [GO:0071988] (biological process) Definition: A process in which a protein is transported to, or maintained at, the spindle pole body. Sources: GOC:mah Relationships: is a type of protein localization to microtubule organizing center [GO:1905508] Regulation: regulated by regulation of protein localization to spindle pole body [GO:1902363]; negatively regulated by negative regulation of protein localization to spindle pole body [GO:1902364]; positively regulated by positive regulation of protein localization to spindle pole body [GO:1902365] Subtypes: establishment of protein localization to spindle pole body [GO:0071989], protein localization to mitotic spindle pole body [GO:1902440], protein localization to meiotic spindle pole body [GO:1902441] Also known as: protein localisation to spindle pole body